{
  "gene": "UniProtKB:Q13459",
  "term_id": "GO:0051015",
  "gene_symbol": "MYO9B",
  "term_label": "actin filament binding",
  "gene_name": "Unconventional myosin-IXb"
}